{
  "gene": "UniProtKB:P12035",
  "term_id": "GO:0045109",
  "gene_symbol": "KRT3",
  "term_label": "intermediate filament organization",
  "gene_name": "Keratin, type II cytoskeletal 3"
}